negative regulation of interleukin-1 beta production [GO:0032691] (biological process) Definition: Any process that stops, prevents, or reduces the frequency, rate, or extent of interleukin-1 beta production. Also known as: down regulation of interleukin-1 beta production, down-regulation of interleukin-1 beta production, downregulation of interleukin-1 beta production, negative regulation of IL-1 beta production, inhibition of interleukin-1 beta production, negative regulation of interleukin-1 beta biosynthetic process, negative regulation of interleukin-1 beta secretion Relationships: is a type of regulation of interleukin-1 beta production [GO:0032651]; is a type of negative regulation of interleukin-1 production [GO:0032692]; negatively regulates interleukin-1 beta production [GO:0032611] Sources: GOC:mah